{
  "gene": "UniProtKB:Q659C4",
  "gene_symbol": "LARP1B",
  "term_id": "GO:0045727",
  "term_label": "positive regulation of translation",
  "gene_name": "La-related protein 1B"
}